{
  "gene": "UniProtKB:P31276",
  "term_label": "DNA-binding transcription factor activity, RNA polymerase II-specific",
  "term_id": "GO:0000981",
  "gene_name": "Homeobox protein Hox-C13",
  "gene_symbol": "HOXC13"
}